{
  "gene": "UniProtKB:O14525",
  "term_id": "GO:0001764",
  "term_label": "neuron migration",
  "gene_symbol": "ASTN1",
  "gene_name": "Astrotactin-1"
}